{
  "term_label": "regulation of RNA splicing",
  "gene_symbol": "HNRNPF",
  "term_id": "GO:0043484",
  "gene_name": "Heterogeneous nuclear ribonucleoprotein F",
  "gene": "UniProtKB:P52597"
}